{
  "gene": "UniProtKB:P13866",
  "gene_symbol": "SLC5A1",
  "term_id": "GO:0098708",
  "term_label": "D-glucose import across plasma membrane",
  "gene_name": "Sodium_glucose cotransporter 1"
}